{
  "gene_symbol": "ARHGEF26",
  "term_label": "guanyl-nucleotide exchange factor activity",
  "term_id": "GO:0005085",
  "gene_name": "Rho guanine nucleotide exchange factor 26",
  "gene": "UniProtKB:Q96DR7"
}